sprouting angiogenesis [GO:0002040] (biological process) Relationships: is a type of GO:0001525 Definition: The extension of new blood vessels from existing vessels into avascular tissues, this process includes the specialization of endothelial cells into leading tip and stalk cells, proliferation and migration of the endothelial cells and cell adhesion resulting in angiogenic sprout fusion or lumen formation. Regulation: RO_0002211 by regulation of sprouting angiogenesis [GO:1903670]; negatively regulated by negative regulation of sprouting angiogenesis [GO:1903671]; positively regulated by GO:1903672 References: PMID:16391003, PMID:23031691